{
  "gene_name": "Protein IMPACT",
  "gene_symbol": "IMPACT",
  "term_id": "GO:0006446",
  "term_label": "regulation of translational initiation",
  "gene": "UniProtKB:Q9P2X3"
}